{
  "gene_symbol": "TMEM205",
  "term_id": "UNKNOWN:0002",
  "term_label": "Unknown biological process",
  "gene_name": "Transmembrane protein 205",
  "gene": "UniProtKB:Q6UW68"
}